{
  "term_id": "GO:0005737",
  "term_label": "cytoplasm",
  "gene_name": "S-phase kinase-associated protein 1",
  "gene": "UniProtKB:P63208",
  "gene_symbol": "SKP1"
}